{
  "gene": "UniProtKB:P14678",
  "term_label": "U5 snRNP",
  "gene_symbol": "SNRPB",
  "term_id": "GO:0005682",
  "gene_name": "Small nuclear ribonucleoprotein-associated proteins B and B'"
}